culmination involved in sorocarp development [GO:0031154] (BP) Definition: The process whose specific outcome is the progression of the culminant over time, from its formation to the mature structure. Culmination begins with a morphogenetic change of the finger-like or migratory slug giving rise to an organized structure containing a stalk and a sorus. This process is the final stage of sorocarp development. Sources: GOC:mah, GOC:mtg_sensu, ISBN:0521583640 Also known as: culminant development, culmination during fruiting body development, culmination during sorocarp development Relationships: is a type of GO:0099120; BFO_0000050 sorocarp development [GO:0030587]